sieve element differentiation [GO:0090603] (biological process) Sources: GOC:tb Subtypes: sieve cell differentiation [GO:0048756] Relationships: is a type of cell differentiation [GO:0030154] Definition: The process whereby a relatively unspecialized cell acquires specialized features of a sieve element.